regulation of cortisol biosynthetic process [GO:2000064] (biological process) Sources: GOC:obol, GOC:yaf Relationships: is a type of regulation of ketone biosynthetic process [GO:0010566]; is a type of regulation of glucocorticoid biosynthetic process [GO:0031946]; is_a regulation of alcohol biosynthetic process [GO:1902930]; regulates cortisol biosynthetic process [GO:0034651] Definition: Any process that modulates the frequency, rate or extent of cortisol biosynthetic process. Subtypes: negative regulation of cortisol biosynthetic process [GO:2000065], positive regulation of cortisol biosynthetic process [GO:2000066] Also known as: regulation of cortisol biosynthesis, regulation of cortisol formation, regulation of cortisol synthesis, regulation of cortisol anabolism